{
  "gene_symbol": "APPBP2",
  "gene": "UniProtKB:Q92624",
  "term_label": "Cul2-RING ubiquitin ligase complex",
  "term_id": "GO:0031462",
  "gene_name": "Amyloid protein-binding protein 2"
}